{
  "gene": "UniProtKB:P0DPK2",
  "gene_symbol": "H3Y1",
  "gene_name": "Histone H3.Y",
  "term_label": "kinetochore",
  "term_id": "GO:0000776"
}